{
  "gene_name": "Bifunctional epoxide hydrolase 2",
  "gene_symbol": "EPHX2",
  "term_id": "GO:0046839",
  "gene": "UniProtKB:P34913",
  "term_label": "phospholipid dephosphorylation"
}